{
  "term_label": "Unknown molecular function",
  "gene_symbol": "WASL",
  "gene": "UniProtKB:O00401",
  "term_id": "UNKNOWN:0001",
  "gene_name": "Actin nucleation-promoting factor WASL"
}